{
  "gene": "UniProtKB:Q12802",
  "term_label": "MAP-kinase scaffold activity",
  "gene_symbol": "AKAP13",
  "gene_name": "A-kinase anchor protein 13",
  "term_id": "GO:0005078"
}